{
  "term_id": "GO:0032266",
  "term_label": "phosphatidylinositol-3-phosphate binding",
  "gene_symbol": "WDR45B",
  "gene_name": "WD repeat domain phosphoinositide-interacting protein 3",
  "gene": "UniProtKB:Q5MNZ6"
}